{
  "term_id": "GO:0032981",
  "gene_symbol": "DMAC1",
  "term_label": "mitochondrial respiratory chain complex I assembly",
  "gene": "UniProtKB:Q96GE9",
  "gene_name": "Distal membrane-arm assembly complex protein 1"
}